{
  "gene_symbol": "FOXA1",
  "gene": "UniProtKB:P55317",
  "term_id": "GO:0000978",
  "term_label": "RNA polymerase II cis-regulatory region sequence-specific DNA binding",
  "gene_name": "Hepatocyte nuclear factor 3-alpha"
}